iron-guanylylpyridinol cofactor biosynthetic process [GO:0160300] (biological process) Also known as: Fe-GP cofactor biosynthetic process References: PMID:37671838 Definition: The chemical reactions and pathways resulting in the formation of iron-guanylylpyridinol cofactor, in which mononuclear Fe(II) is ligated with a pyridinol and two CO ligands. Relationships: is a type of biosynthetic process [GO:0009058]